{
  "term_id": "UNKNOWN:0003",
  "gene_symbol": "TRBJ2-2P",
  "gene": "UniProtKB:A0A0A0MTA2",
  "term_label": "Unknown cellular component",
  "gene_name": "T cell receptor beta joining 2-2P (non-functional) (Fragment)"
}